{
  "gene_name": "Sphingosine-1-phosphate phosphatase 1",
  "gene": "UniProtKB:Q9BX95",
  "gene_symbol": "SGPP1",
  "term_label": "sphingosine-1-phosphate phosphatase activity",
  "term_id": "GO:0042392"
}